{
  "term_label": "NADP+ metabolic process",
  "term_id": "GO:0006739",
  "gene": "UniProtKB:P48735",
  "gene_name": "Isocitrate dehydrogenase [NADP], mitochondrial",
  "gene_symbol": "IDH2"
}